{
  "gene_name": "Olfactory receptor 1D4",
  "term_id": "GO:0004984",
  "term_label": "olfactory receptor activity",
  "gene": "UniProtKB:P47884",
  "gene_symbol": "OR1D4"
}